L-serine catabolic process [GO:0006565] (biological process) Definition: The chemical reactions and pathways resulting in the breakdown of L-serine, the L-enantiomer of serine, i.e. (2S)-2-amino-3-hydroxypropanoic acid. Sources: GOC:ai, GOC:jsg Also known as: L-serine breakdown, L-serine catabolism, L-serine degradation Relationships: is a type of L-serine metabolic process [GO:0006563]; is a type of L-amino acid catabolic process [GO:0170035]; is a type of proteinogenic amino acid catabolic process [GO:0170040]